regulation of nuclear cell cycle DNA replication [GO:0033262] (biological process) Also known as: regulation of DNA replication involved in S phase, regulation of DNA replication involved in S-phase, regulation of DNA replication during S phase Relationships: is a type of regulation of cell cycle process [GO:0010564]; is a type of regulation of DNA-templated DNA replication [GO:0090329]; regulates nuclear DNA replication [GO:0033260] Subtypes: positive regulation of nuclear cell cycle DNA replication [GO:0010571], negative regulation of nuclear cell cycle DNA replication [GO:1902576], GO:1903463, regulation of initiation of premeiotic DNA replication [GO:1904512] Sources: GOC:mtg_cell_cycle Definition: Any process that modulates the frequency, rate or extent of The DNA-dependent DNA replication that occurs in the nucleus of eukaryotic organisms as part of the cell cycle.